{
  "gene_name": "HCLS1-associated protein X-1",
  "term_label": "mitochondrion",
  "gene": "UniProtKB:O00165",
  "gene_symbol": "HAX1",
  "term_id": "GO:0005739"
}